magnetoreception by sensory perception of mechanical stimulus [GO:0050979] (biological process) Also known as: magnetoreception through mechanical stimulus, magnetoreception, sensory perception of mechanical stimulus, magnetoreception, using mechanical stimulus Relationships: is a type of sensory perception of mechanical stimulus [GO:0050954]; is a type of magnetoreception [GO:0050958] References: PMID:15886990 Sources: GOC:ai, Wikipedia:Magnetoception Definition: The series of events required for an organism to receive a mechanical stimulus relating to a magnetic field, convert it to a molecular signal, and recognize and characterize the signal. A magnetic field exerts a torque on a ferromagnetic material (e.g. magnetite) or on a material with diamagnetic anisotropy; organisms that can detect this torque can use it to determine the orientation of the magnetic field.